cinnamic acid metabolic process [GO:0009803] (biological process) Subtypes: cinnamic acid biosynthetic process [GO:0009800], cinnamic acid catabolic process [GO:0046281] Definition: The chemical reactions and pathways involving cinnamic acid, 3-phenyl-2-propenoic acid. Also known as: cinnamic acid metabolism, cinnamylic acid metabolic process, cinnamylic acid metabolism, phenylacrylic acid metabolic process, phenylacrylic acid metabolism, phenylpropenoic acid metabolic process, phenylpropenoic acid metabolism Sources: GOC:jl Relationships: is a type of phenylpropanoid metabolic process [GO:0009698]; is a type of GO:0032787; is a type of benzene-containing compound metabolic process [GO:0042537]; is a type of olefinic compound metabolic process [GO:0120254]